{
  "term_id": "GO:0071363",
  "gene_symbol": "AMHR2",
  "gene_name": "Anti-Muellerian hormone type-2 receptor",
  "gene": "UniProtKB:Q16671",
  "term_label": "cellular response to growth factor stimulus"
}